{
  "term_label": "U5 snRNA binding",
  "gene_symbol": "EFTUD2",
  "term_id": "GO:0030623",
  "gene": "UniProtKB:Q15029",
  "gene_name": "116 kDa U5 small nuclear ribonucleoprotein component"
}